{
  "term_label": "protein refolding",
  "term_id": "GO:0042026",
  "gene": "UniProtKB:P48741",
  "gene_name": "Putative heat shock 70 kDa protein 7",
  "gene_symbol": "HSPA7"
}